{
  "term_id": "GO:0034599",
  "gene_name": "Fanconi anemia group C protein",
  "gene": "UniProtKB:Q00597",
  "gene_symbol": "FANCC",
  "term_label": "cellular response to oxidative stress"
}